{
  "gene_symbol": "TCAF1",
  "gene_name": "TRPM8 channel-associated factor 1",
  "gene": "UniProtKB:Q9Y4C2",
  "term_label": "plasma membrane",
  "term_id": "GO:0005886"
}